viral replication complex [GO:0019034] (cellular component) Definition: Specific locations and structures in the virus infected cell involved in replicating the viral genome. Relationships: is a type of GO:0044094 Sources: ISBN:0781718325